{
  "term_id": "GO:0051371",
  "term_label": "muscle alpha-actinin binding",
  "gene_symbol": "PKD2L1",
  "gene_name": "Polycystin-2-like protein 1",
  "gene": "UniProtKB:Q9P0L9"
}